{
  "term_id": "GO:0045727",
  "gene": "UniProtKB:Q9H1J1",
  "gene_symbol": "UPF3A",
  "gene_name": "Regulator of nonsense transcripts 3A",
  "term_label": "positive regulation of translation"
}